{
  "gene_name": "Rho-related GTP-binding protein RhoJ",
  "term_label": "establishment of cell polarity",
  "gene": "UniProtKB:Q9H4E5",
  "term_id": "GO:0030010",
  "gene_symbol": "RHOJ"
}